{
  "gene_name": "Lysine-specific demethylase 9",
  "gene_symbol": "RSBN1",
  "term_id": "GO:0005634",
  "gene": "UniProtKB:Q5VWQ0",
  "term_label": "nucleus"
}